{
  "term_label": "Unknown biological process",
  "term_id": "UNKNOWN:0002",
  "gene_name": "Beta-defensin 107",
  "gene": "UniProtKB:Q8IZN7",
  "gene_symbol": "DEFB107A"
}